{
  "gene": "UniProtKB:Q6DHV5",
  "gene_symbol": "CC2D2B",
  "gene_name": "Protein CC2D2B",
  "term_id": "GO:1904491",
  "term_label": "protein localization to ciliary transition zone"
}